{
  "gene_symbol": "DMRTA1",
  "term_id": "GO:0007548",
  "term_label": "sex differentiation",
  "gene_name": "Doublesex- and mab-3-related transcription factor A1",
  "gene": "UniProtKB:Q5VZB9"
}